renal phosphate ion absorption [GO:0097291] (biological process) Also known as: renal phosphate absorption References: PMID:18784102, PMID:22506049 Sources: GOC:lb Definition: A renal system process in which phosphate ions are taken up from the collecting ducts and proximal and distal loops of the nephron. In non-mammalian species, absorption may occur in related structures. Relationships: is a type of GO:0070293